immune response-activating cell surface receptor signaling pathway [GO:0002429] (biological process) Relationships: is a type of immune response-activating signaling pathway [GO:0002757]; is a type of immune response-regulating cell surface receptor signaling pathway [GO:0002768] Subtypes: innate immune response activating cell surface receptor signaling pathway [GO:0002220], complement receptor mediated signaling pathway [GO:0002430], Fc receptor mediated stimulatory signaling pathway [GO:0002431], antigen receptor-mediated signaling pathway [GO:0050851] Definition: The series of molecular signals initiated by an extracellular ligand binding to a receptor on the surface of a cell, leading to the activation or perpetuation of an immune response. Sources: GOC:add, GO_REF:0000022, ISBN:0781735149 Also known as: activation of immune response by cell surface receptor signaling pathway, immune response-activating cell surface receptor signalling pathway